{
  "gene_symbol": "PARD3B",
  "term_label": "adherens junction",
  "gene_name": "Partitioning defective 3 homolog B",
  "term_id": "GO:0005912",
  "gene": "UniProtKB:Q8TEW8"
}